{
  "gene_name": "Prolyl endopeptidase",
  "gene_symbol": "PREP",
  "term_id": "GO:0005829",
  "gene": "UniProtKB:P48147",
  "term_label": "cytosol"
}